L-glutamate biosynthetic process [GO:0097054] (biological process) Sources: GOC:yaf Definition: The chemical reactions and pathways resulting in the formation of L-glutamate, the L enantiomer anion of 2-aminopentanedioic acid. Relationships: is a type of GO:0006537 Also known as: L-glutamate anabolism, L-glutamate biosynthesis, L-glutamate formation, L-glutamate synthesis